{
  "term_label": "actin filament debranching",
  "gene": "UniProtKB:O60234",
  "gene_symbol": "GMFG",
  "term_id": "GO:0071846",
  "gene_name": "Glia maturation factor gamma"
}